{
  "gene": "UniProtKB:Q9NQS5",
  "gene_symbol": "GPR84",
  "gene_name": "G-protein coupled receptor 84",
  "term_label": "neuropeptide signaling pathway",
  "term_id": "GO:0007218"
}